{
  "term_id": "GO:0005802",
  "gene": "UniProtKB:Q8TF62",
  "term_label": "trans-Golgi network",
  "gene_symbol": "ATP8B4",
  "gene_name": "Probable phospholipid-transporting ATPase IM"
}